raffinose transmembrane transporter activity [GO:0015158] (molecular function) Sources: GOC:mtg_transport, ISBN:0198506732, ISBN:0815340729 Definition: Enables the transfer of raffinose from one side of a membrane to the other. Raffinose occurs in plants almost as commonly as sucrose and is present in cereal grains, cotton seeds, and many legumes. It is synthesized from sucrose by transfer of a galactopyranoside from myo-inositol. Subtypes: GO:0015529 Also known as: raffinose permease Relationships: is a type of oligosaccharide transmembrane transporter activity [GO:0015157]; BFO_0000050 raffinose transport [GO:0015773]